{
  "gene_symbol": "WIPF3",
  "term_id": "GO:0006887",
  "gene_name": "WAS_WASL-interacting protein family member 3",
  "gene": "UniProtKB:A6NGB9",
  "term_label": "exocytosis"
}